{
  "gene": "UniProtKB:Q15744",
  "term_label": "myeloid cell differentiation",
  "gene_name": "CCAAT_enhancer-binding protein epsilon",
  "term_id": "GO:0030099",
  "gene_symbol": "CEBPE"
}